symbiotic process benefiting host [GO:0085030] (biological process) Definition: A process carried out by symbiont gene products that enables a symbiotic interaction with a host organism, that is beneficial to the host organism. Sources: GOC:pdt Also known as: mutualism Relationships: is a type of biological process involved in symbiotic interaction [GO:0044403]